{
  "gene_symbol": "RPL17",
  "term_label": "structural constituent of ribosome",
  "term_id": "GO:0003735",
  "gene_name": "Large ribosomal subunit protein uL22",
  "gene": "UniProtKB:P18621"
}